{
  "term_id": "UNKNOWN:0002",
  "gene_name": "UPF0728 protein C10orf53",
  "term_label": "Unknown biological process",
  "gene_symbol": "C10orf53",
  "gene": "UniProtKB:Q8N6V4"
}